{
  "gene_symbol": "ABI2",
  "gene": "UniProtKB:Q9NYB9",
  "gene_name": "Abl interactor 2",
  "term_label": "lamellipodium",
  "term_id": "GO:0030027"
}